{
  "gene": "UniProtKB:Q96KJ9",
  "gene_name": "Cytochrome c oxidase subunit 4 isoform 2, mitochondrial",
  "term_label": "mitochondrial electron transport, cytochrome c to oxygen",
  "term_id": "GO:0006123",
  "gene_symbol": "COX4I2"
}